{
  "gene_symbol": "PTEN",
  "term_id": "GO:0042995",
  "gene_name": "Phosphatidylinositol 3,4,5-trisphosphate 3-phosphatase and dual-specificity protein phosphatase PTEN",
  "gene": "UniProtKB:P60484",
  "term_label": "cell projection"
}